{
  "term_id": "GO:0006506",
  "term_label": "GPI anchor biosynthetic process",
  "gene": "UniProtKB:Q92521",
  "gene_name": "GPI mannosyltransferase 3",
  "gene_symbol": "PIGB"
}